{
  "term_id": "GO:0006281",
  "gene_name": "Serine_threonine-protein kinase ATR",
  "gene": "UniProtKB:Q13535",
  "term_label": "DNA repair",
  "gene_symbol": "ATR"
}